{
  "gene_symbol": "GSDMB",
  "term_id": "GO:0070273",
  "gene_name": "Gasdermin-B",
  "term_label": "phosphatidylinositol-4-phosphate binding",
  "gene": "UniProtKB:Q8TAX9"
}